acetate transmembrane transport [GO:0035433] (biological process) Note: Note that this term is not intended for use in annotating lateral movement within membranes. Sources: GOC:vw Definition: The process in which acetate is transported across a membrane. Acetate is the 2-carbon carboxylic acid ethanoic acid. Relationships: is a type of acetate transport [GO:0006846]; is a type of carboxylic acid transmembrane transport [GO:1905039] Also known as: acetate membrane transport Subtypes: plasma membrane acetate transport [GO:0006847]